{
  "gene": "UniProtKB:Q9H6Z9",
  "term_label": "ferrous iron binding",
  "gene_name": "Prolyl hydroxylase EGLN3",
  "term_id": "GO:0008198",
  "gene_symbol": "EGLN3"
}